{
  "gene": "UniProtKB:Q6PJG2",
  "gene_name": "Mitotic deacetylase-associated SANT domain protein",
  "term_id": "GO:0045892",
  "gene_symbol": "MIDEAS",
  "term_label": "negative regulation of DNA-templated transcription"
}